protein-disulfide reductase (glutathione) activity [GO:0019153] (molecular function) Also known as: protein-disulphide reductase (glutathione) activity, glutathione-insulin transhydrogenase activity, insulin reductase activity, glutaredoxin reductase, protein disulfide reductase (glutathione), protein disulfide transhydrogenase activity Definition: Catalysis of the reaction: 2 glutathione + protein-disulfide = glutathione disulfide+ protein-dithiol. Relationships: is a type of protein-disulfide reductase activity [GO:0015035]; is a type of oxidoreductase activity, acting on a sulfur group of donors, disulfide as acceptor [GO:0016671] Sources: RHEA:21064